tubulin binding [GO:0015631] (molecular function) Sources: GOC:clt Definition: Binding to monomeric or multimeric forms of tubulin, including microtubules. Relationships: is a type of cytoskeletal protein binding [GO:0008092] Subtypes: microtubule binding [GO:0008017], alpha-tubulin binding [GO:0043014], gamma-tubulin binding [GO:0043015], GO:0048487